regulation of response to wounding [GO:1903034] (biological process) Relationships: is a type of regulation of response to stress [GO:0080134]; regulates response to wounding [GO:0009611] References: PMID:19164535 Sources: GOC:TermGenie, GOC:kmv, GO_REF:0000058 Also known as: regulation of physiological response to wounding Subtypes: regulation of axon regeneration [GO:0048679], regulation of wound healing [GO:0061041], regulation of inflammatory response to wounding [GO:0106014], negative regulation of response to wounding [GO:1903035], positive regulation of response to wounding [GO:1903036] Definition: Any process that modulates the frequency, rate or extent of response to wounding.